{
  "gene_name": "Putative inactive neutral ceramidase B",
  "term_id": "UNKNOWN:0001",
  "gene_symbol": "ASAH2B",
  "term_label": "Unknown molecular function",
  "gene": "UniProtKB:P0C7U1"
}